{
  "term_id": "GO:0009986",
  "gene_symbol": "ITGA3",
  "term_label": "cell surface",
  "gene": "UniProtKB:P26006",
  "gene_name": "Integrin alpha-3"
}